{
  "gene": "UniProtKB:Q6PH85",
  "gene_symbol": "DCUN1D2",
  "gene_name": "DCN1-like protein 2",
  "term_label": "cullin family protein binding",
  "term_id": "GO:0097602"
}